{
  "gene": "UniProtKB:Q92839",
  "term_label": "plasma membrane",
  "gene_symbol": "HAS1",
  "term_id": "GO:0005886",
  "gene_name": "Hyaluronan synthase 1"
}